4-hydroxybenzoyl-CoA reductase activity [GO:0018525] (molecular function) Sources: RHEA:29603 Relationships: is a type of GO:0016636 Definition: Catalysis of the reaction: benzoyl-CoA + oxidized ferredoxin + H2O = 4-hydroxybenzoyl-CoA + reduced ferredoxin. Also known as: 4-hydroxybenzoyl-coA reductase (dehydroxylating) activity, 4-hydroxybenzoyl-coA:(acceptor) oxidoreductase activity